glycerophospholipid arachidonoyl-transferase (CoA-independent) activity [GO:0047177] (molecular function) Definition: Catalysis of the reaction: 1-alkyl-2-lyso-sn-glycero-3-phosphoethanolamine + 1-alkyl-2-arachidonyl-sn-glycero-3-phosphocholine = 1-alkyl-2-lyso-sn-glycero-3-phosphocholine + 1-alkyl-2-arachidonyl-sn-glycero-3-phosphoethanolamine. Sources: EC:2.3.1.147, MetaCyc:2.3.1.147-RXN Also known as: 1-organyl-2-arachidonoyl-sn-glycero-3-phosphocholine:1-organyl-2-lyso-sn-glycero-3-phosphoethanolamine arachidonoyltransferase (CoA-independent), 1-organyl-2-arachidonyl-sn-glycero-3-phosphocholine:1-organyl-2-lyso-sn-glycero-3-phosphoethanolamine arachidonoyltransferase (CoA-independent) Relationships: is a type of acyltransferase activity, transferring groups other than amino-acyl groups [GO:0016747]